{
  "gene": "UniProtKB:Q96BY7",
  "term_label": "phosphatidylinositol-3-phosphate binding",
  "term_id": "GO:0032266",
  "gene_symbol": "ATG2B",
  "gene_name": "Autophagy-related protein 2 homolog B"
}